nucleotide biosynthetic process [GO:0009165] (biological process) Subtypes: purine nucleotide biosynthetic process [GO:0006164], GO:0006221, cyclic nucleotide biosynthetic process [GO:0009190], ribonucleotide biosynthetic process [GO:0009260], deoxyribonucleotide biosynthetic process [GO:0009263], bis(5'-nucleosidyl) oligophosphate biosynthetic process [GO:0015957], GO:0015960, pyridine nucleotide biosynthetic process [GO:0019363], GO:0043173, GO:0046940, flavin adenine dinucleotide biosynthetic process [GO:0072388], GO:1902758 Also known as: nucleotide anabolism, nucleotide biosynthesis, nucleotide formation, nucleotide synthesis Sources: GOC:go_curators Regulation: regulated by GO:0030808; negatively regulated by negative regulation of nucleotide biosynthetic process [GO:0030809]; RO_0002213 by GO:0030810 Definition: The chemical reactions and pathways resulting in the formation of nucleotides, any nucleoside that is esterified with (ortho)phosphate or an oligophosphate at any hydroxyl group on the glycose moiety; may be mono-, di- or triphosphate; this definition includes cyclic-nucleotides (nucleoside cyclic phosphates). Relationships: is_a nucleotide metabolic process [GO:0009117]; is a type of GO:1901293